{
  "gene_symbol": "ABTB1",
  "gene_name": "Ankyrin repeat and BTB_POZ domain-containing protein 1",
  "term_id": "UNKNOWN:0001",
  "term_label": "Unknown molecular function",
  "gene": "UniProtKB:Q969K4"
}